17(E)-cheilanthenediol synthase activity [GO:0102645] (molecular function) Relationships: is a type of hydro-lyase activity [GO:0016836] References: PMID:24200803 Sources: GOC:pz Definition: Catalysis of the reaction: 17(E)-cheilanthenediol = all-trans-geranylfarnesol + H2O.